{
  "term_label": "auditory receptor cell morphogenesis",
  "gene": "UniProtKB:Q9Y6N9",
  "gene_name": "Harmonin",
  "gene_symbol": "USH1C",
  "term_id": "GO:0002093"
}